{
  "gene_symbol": "DOCK8",
  "gene_name": "Dedicator of cytokinesis protein 8",
  "gene": "UniProtKB:Q8NF50",
  "term_id": "GO:1903905",
  "term_label": "positive regulation of establishment of T cell polarity"
}